{
  "term_id": "GO:0005251",
  "term_label": "delayed rectifier potassium channel activity",
  "gene_symbol": "KCNE2",
  "gene_name": "Potassium voltage-gated channel subfamily E member 2",
  "gene": "UniProtKB:Q9Y6J6"
}